{
  "gene_symbol": "TRAJ35",
  "gene_name": "T cell receptor alpha joining 35 (non-functional) (Fragment)",
  "term_id": "UNKNOWN:0003",
  "gene": "UniProtKB:A0A075B6Y2",
  "term_label": "Unknown cellular component"
}